{
  "gene": "UniProtKB:A8MQT2",
  "term_id": "GO:0000137",
  "term_label": "Golgi cis cisterna",
  "gene_symbol": "GOLGA8B",
  "gene_name": "Golgin subfamily A member 8B"
}